meiosis I cell cycle process [GO:0061982] (biological process) Definition: A process that contributes to the first meiotic division. The first meiotic division is the reductive division resulting in the separation of homologous chromosome pairs. Subtypes: meiotic DNA recombinase assembly [GO:0000707], meiotic strand invasion [GO:0000708], GO:0000710, meiotic DNA repair synthesis [GO:0000711], resolution of meiotic recombination intermediates [GO:0000712], meiotic heteroduplex formation [GO:0000713], meiotic strand displacement [GO:0000714], GO:0006311, GO:0007110, GO:0007127, G2/MI transition of meiotic cell cycle [GO:0008315], meiotic DNA double-strand break formation [GO:0042138], karyosome formation [GO:0061988], metaphase/anaphase transition of meiosis I [GO:1990949] Also known as: first meiotic cell division Relationships: is a type of meiotic cell cycle process [GO:1903046] References: PMID:29385397